{
  "gene_symbol": "MYCBPAP",
  "gene_name": "MYCBP-associated protein",
  "term_id": "GO:0005886",
  "term_label": "plasma membrane",
  "gene": "UniProtKB:Q8TBZ2"
}